{
  "gene": "UniProtKB:Q9H469",
  "term_label": "SCF-dependent proteasomal ubiquitin-dependent protein catabolic process",
  "term_id": "GO:0031146",
  "gene_name": "F-box_LRR-repeat protein 15",
  "gene_symbol": "FBXL15"
}